microcin B17 transport [GO:0042885] (biological process) Definition: The directed movement of microcin B17, a bactericidal peptide (antibiotic) produced by some enteric bacteria, into, out of or within a cell, or between cells, by means of some agent such as a transporter or pore. Relationships: is a type of microcin transport [GO:0042884] References: PMID:11292337 Sources: GOC:jl